{
  "gene_name": "PRKR-interacting protein 1",
  "gene_symbol": "PRKRIP1",
  "term_id": "GO:0019901",
  "gene": "UniProtKB:Q9H875",
  "term_label": "protein kinase binding"
}